tetraspanin-enriched microdomain [GO:0097197] (CC) Relationships: is a type of cellular anatomical structure [GO:0110165]; is part of plasma membrane [GO:0005886] Also known as: TEM, membrane tetraspanin-enriched microdomain Definition: A pre-organized unit composed either of adhesion molecules (mainly integrins and members of the Ig superfamily), signaling receptors and/or enzyme-enriched plasma membrane domains that compartmentalizes cellular processes. Tetraspanin-enriched microdomains might be specially suited for the regulation of avidity of adhesion receptors and the compartmentalization of enzymatic activities. References: PMID:19709882, PMID:21930792 Sources: GOC:ans